{
  "gene_symbol": "FLG2",
  "term_label": "cornified envelope",
  "gene_name": "Filaggrin-2",
  "gene": "UniProtKB:Q5D862",
  "term_id": "GO:0001533"
}